glycerol dehydrogenase (NADP+) activity [GO:0047956] (molecular function) Sources: RHEA:23592 Relationships: is a type of oxidoreductase activity, acting on the CH-OH group of donors, NAD or NADP as acceptor [GO:0016616] Definition: Catalysis of the reaction: glycerol + NADP+ = D-glyceraldehyde + NADPH. Also known as: glycerol dehydrogenase [NADP+] activity, glycerol:NADP+ oxidoreductase activity